{
  "gene_symbol": "SAYSD1",
  "gene_name": "SAYSvFN domain-containing protein 1",
  "term_id": "GO:0072344",
  "term_label": "rescue of stalled ribosome",
  "gene": "UniProtKB:Q9NPB0"
}